kininogen binding [GO:0030984] (molecular function) Definition: Binding to a kininogen, a kinin precursor. Relationships: is a type of protein binding [GO:0005515] References: PMID:9520414 Sources: GOC:mah Subtypes: GO:0030985, GO:0030986